{
  "gene_symbol": "PRDX1",
  "term_label": "leukocyte activation",
  "term_id": "GO:0045321",
  "gene": "UniProtKB:Q06830",
  "gene_name": "Peroxiredoxin-1"
}